{
  "gene_symbol": "ASH1L",
  "term_id": "GO:0042800",
  "term_label": "histone H3K4 methyltransferase activity",
  "gene": "UniProtKB:Q9NR48",
  "gene_name": "Histone-lysine N-methyltransferase ASH1L"
}